{
  "gene": "UniProtKB:P31949",
  "term_id": "UNKNOWN:0002",
  "gene_name": "Protein S100-A11",
  "gene_symbol": "S100A11",
  "term_label": "Unknown biological process"
}